{
  "term_id": "GO:0003712",
  "gene_symbol": "ZNF653",
  "gene": "UniProtKB:Q96CK0",
  "gene_name": "Zinc finger protein 653",
  "term_label": "transcription coregulator activity"
}